{
  "gene_symbol": "RNF186",
  "term_id": "GO:0035519",
  "gene": "UniProtKB:Q9NXI6",
  "term_label": "protein K29-linked ubiquitination",
  "gene_name": "E3 ubiquitin-protein ligase RNF186"
}